{
  "term_id": "GO:0031209",
  "gene_name": "Actin-binding protein WASF2",
  "gene": "UniProtKB:Q9Y6W5",
  "term_label": "SCAR complex",
  "gene_symbol": "WASF2"
}